{
  "gene": "UniProtKB:Q6P9B9",
  "gene_name": "Integrator complex subunit 5",
  "gene_symbol": "INTS5",
  "term_id": "GO:0032039",
  "term_label": "integrator complex"
}